{
  "term_id": "UNKNOWN:0003",
  "gene_name": "Putative ATP synthase subunit g 2, mitochondrial",
  "term_label": "Unknown cellular component",
  "gene_symbol": "ATP5MGL",
  "gene": "UniProtKB:Q7Z4Y8"
}